{
  "gene_symbol": "PRDX1",
  "term_id": "GO:0006979",
  "gene": "UniProtKB:Q06830",
  "gene_name": "Peroxiredoxin-1",
  "term_label": "response to oxidative stress"
}